{
  "gene_name": "BTB_POZ domain-containing protein KCTD7",
  "gene": "UniProtKB:Q96MP8",
  "term_label": "plasma membrane",
  "term_id": "GO:0005886",
  "gene_symbol": "KCTD7"
}